{
  "gene": "UniProtKB:P13533",
  "gene_symbol": "MYH6",
  "term_label": "myosin filament",
  "term_id": "GO:0032982",
  "gene_name": "Myosin-6"
}